positive regulation of free ubiquitin chain polymerization [GO:1904544] (biological process) References: PMID:24660806 Sources: GOC:PARL, GOC:TermGenie, GOC:pad, GO_REF:0000058 Also known as: up regulation of free ubiquitin chain polymerization, up-regulation of free ubiquitin chain polymerization, upregulation of free ubiquitin chain polymerization, activation of free ubiquitin chain polymerization Note: An example of this is PARK2 in human (UniProt symbol O60260) in PMID:24660806 (inferred from mutant phenotype). Relationships: is_a positive regulation of protein polymerization [GO:0032273]; is a type of regulation of free ubiquitin chain polymerization [GO:1904542]; positively regulates GO:0010994 Definition: Any process that activates or increases the frequency, rate or extent of free ubiquitin chain polymerization.